{
  "term_label": "heterochromatin formation",
  "term_id": "GO:0031507",
  "gene_name": "DNA polymerase epsilon subunit 3",
  "gene_symbol": "POLE3",
  "gene": "UniProtKB:Q9NRF9"
}